hedgehog family protein binding [GO:0097108] (molecular function) Definition: Binding to a member of the hedgehog protein family, signaling proteins involved in development. References: PMID:10050855 Sources: GOC:BHF, GOC:pr Relationships: is a type of GO:0005515